{
  "term_id": "GO:0005737",
  "term_label": "cytoplasm",
  "gene_name": "Protein kinase C and casein kinase substrate in neurons protein 3",
  "gene": "UniProtKB:Q9UKS6",
  "gene_symbol": "PACSIN3"
}